{
  "term_id": "UNKNOWN:0001",
  "gene_name": "Trinucleotide repeat-containing gene 6C protein",
  "gene": "UniProtKB:Q9HCJ0",
  "term_label": "Unknown molecular function",
  "gene_symbol": "TNRC6C"
}